negative regulation of protein localization to spindle pole body [GO:1902364] (BP) Definition: Any process that stops, prevents or reduces the frequency, rate or extent of protein localization to spindle pole body. Subtypes: negative regulation of protein localization to meiotic spindle pole body [GO:0140435], negative regulation of protein localization to mitotic spindle pole body [GO:1902543] Also known as: down regulation of protein localisation to spindle pole body, down regulation of protein localization to spindle pole body, down-regulation of protein localisation to spindle pole body, down-regulation of protein localization to spindle pole body, downregulation of protein localisation to spindle pole body, downregulation of protein localization to spindle pole body, negative regulation of protein localisation to spindle pole body, inhibition of protein localisation to spindle pole body, inhibition of protein localization to spindle pole body Relationships: is a type of regulation of protein localization to spindle pole body [GO:1902363]; is a type of negative regulation of protein localization [GO:1903828]; negatively regulates protein localization to spindle pole body [GO:0071988] References: PMID:21131906 Sources: GOC:TermGenie